taste bud development [GO:0061193] (biological process) Sources: GOC:dph Relationships: is a type of sensory organ development [GO:0007423]; is part of GO:0043586 Definition: The progression of the taste bud over time, from its formation to the mature state. The taste bud is a specialized area of the tongue that contains taste receptors.